protein phosphatase 2A binding [GO:0051721] (molecular function) Relationships: is a type of protein phosphatase binding [GO:0019903] Sources: GOC:ai Also known as: protein phosphatase 2 binding Definition: Binding to protein phosphatase 2A.